{
  "gene_symbol": "IGF2BP2",
  "gene": "UniProtKB:Q9Y6M1",
  "gene_name": "Insulin-like growth factor 2 mRNA-binding protein 2",
  "term_label": "nervous system development",
  "term_id": "GO:0007399"
}